{
  "gene": "UniProtKB:Q96Q07",
  "gene_name": "BTB_POZ domain-containing protein 9",
  "term_label": "cytoplasm",
  "gene_symbol": "BTBD9",
  "term_id": "GO:0005737"
}